{
  "gene": "UniProtKB:O95707",
  "gene_symbol": "POP4",
  "term_id": "GO:0030677",
  "term_label": "ribonuclease P complex",
  "gene_name": "Ribonuclease P protein subunit p29"
}